{
  "term_label": "extracellular space",
  "term_id": "GO:0005615",
  "gene": "UniProtKB:Q86WN2",
  "gene_name": "Interferon epsilon",
  "gene_symbol": "IFNE"
}